{
  "gene_symbol": "CCDC38",
  "gene_name": "Coiled-coil domain-containing protein 38",
  "gene": "UniProtKB:Q502W7",
  "term_id": "GO:0005813",
  "term_label": "centrosome"
}